{
  "term_id": "GO:0070878",
  "gene": "UniProtKB:Q8WYQ5",
  "term_label": "primary miRNA binding",
  "gene_symbol": "DGCR8",
  "gene_name": "Microprocessor complex subunit DGCR8"
}